{
  "term_id": "GO:0005096",
  "term_label": "GTPase activator activity",
  "gene_symbol": "NF1",
  "gene_name": "Neurofibromin",
  "gene": "UniProtKB:P21359"
}